{
  "term_label": "lysosomal membrane",
  "gene": "UniProtKB:Q9NUM4",
  "term_id": "GO:0005765",
  "gene_name": "Transmembrane protein 106B",
  "gene_symbol": "TMEM106B"
}